{
  "term_id": "UNKNOWN:0002",
  "gene_symbol": "PABPC3",
  "gene": "UniProtKB:Q9H361",
  "gene_name": "Polyadenylate-binding protein 3",
  "term_label": "Unknown biological process"
}